{
  "term_id": "GO:0045031",
  "gene_symbol": "P2RY1",
  "term_label": "G protein-coupled ATP receptor activity",
  "gene_name": "P2Y purinoceptor 1",
  "gene": "UniProtKB:P47900"
}